{
  "gene": "UniProtKB:Q9H0E9",
  "gene_name": "Bromodomain-containing protein 8",
  "term_label": "Unknown molecular function",
  "gene_symbol": "BRD8",
  "term_id": "UNKNOWN:0001"
}